{
  "gene_name": "Homeobox protein SIX6",
  "term_id": "GO:0005667",
  "gene": "UniProtKB:O95475",
  "term_label": "transcription regulator complex",
  "gene_symbol": "SIX6"
}